cellular response to silver ion [GO:0071292] (biological process) Definition: Any process that results in a change in state or activity of a cell (in terms of movement, secretion, enzyme production, gene expression, etc.) as a result of a silver (Ag+) ion stimulus. Sources: GOC:mah Relationships: is_a response to silver ion [GO:0010272]; is a type of GO:0071248